complement activation, lectin pathway [GO:0001867] (biological process) Relationships: is a type of complement activation [GO:0006956]; is a type of innate immune response [GO:0045087] Also known as: complement cascade, lectin pathway Regulation: RO_0002211 by regulation of complement activation, lectin pathway [GO:0001868]; negatively regulated by GO:0001869; positively regulated by positive regulation of complement activation, lectin pathway [GO:0001870] Note: Note that proteins such as mannose-binding lectin (MBL) and certain serum ficolins can activate the lectin complement pathway. Sources: GOC:add, ISBN:0781735149 Definition: Any process involved in the activation of any of the steps of the lectin pathway of the complement cascade which allows for the direct killing of microbes and the regulation of other immune processes.